{
  "term_id": "GO:0005886",
  "gene_name": "Alpha-1A adrenergic receptor",
  "term_label": "plasma membrane",
  "gene": "UniProtKB:P35348",
  "gene_symbol": "ADRA1A"
}